{
  "gene_name": "Calcium uptake protein 1, mitochondrial",
  "term_id": "GO:0051560",
  "term_label": "mitochondrial calcium ion homeostasis",
  "gene": "UniProtKB:Q9BPX6",
  "gene_symbol": "MICU1"
}